{
  "gene_name": "WD repeat-containing protein 7",
  "gene": "UniProtKB:Q9Y4E6",
  "term_label": "Unknown molecular function",
  "term_id": "UNKNOWN:0001",
  "gene_symbol": "WDR7"
}